{
  "term_id": "GO:0005634",
  "gene_symbol": "RPS27A",
  "gene_name": "Ubiquitin-ribosomal protein eS31 fusion protein",
  "gene": "UniProtKB:P62979",
  "term_label": "nucleus"
}